{
  "gene_symbol": "FAM169BP",
  "term_id": "UNKNOWN:0003",
  "gene": "UniProtKB:Q8N8A8",
  "gene_name": "Protein FAM169BP",
  "term_label": "Unknown cellular component"
}